{
  "term_id": "GO:0030672",
  "term_label": "synaptic vesicle membrane",
  "gene": "UniProtKB:Q96LB4",
  "gene_symbol": "ATP6V1G3",
  "gene_name": "V-type proton ATPase subunit G 3"
}